mesenchymal cell apoptotic process [GO:0097152] (biological process) Subtypes: mesenchymal cell apoptotic process involved in metanephros development [GO:1900200], mesenchymal cell apoptotic process involved in nephron morphogenesis [GO:1901145] Regulation: regulated by GO:2001053; RO_0002212 by GO:2001054; positively regulated by positive regulation of mesenchymal cell apoptotic process [GO:2001055] Definition: Any apoptotic process in a mesenchymal cell. A mesenchymal cell is a loosely associated cell that is part of the connective tissue in an organism. Mesenchymal cells give rise to more mature connective tissue cell types. References: PMID:18231833 Sources: CL:0000134, GOC:mtg_apoptosis, GOC:yaf Relationships: is a type of apoptotic process [GO:0006915] Also known as: mesenchymal cell apoptosis